{
  "gene_name": "Monoacylglycerol lipase ABHD2",
  "gene_symbol": "ABHD2",
  "term_id": "GO:0046464",
  "term_label": "acylglycerol catabolic process",
  "gene": "UniProtKB:P08910"
}